{
  "term_id": "GO:0072488",
  "gene_symbol": "RHD",
  "gene_name": "Blood group Rh(D) polypeptide",
  "term_label": "ammonium transmembrane transport",
  "gene": "UniProtKB:Q02161"
}